{
  "gene_name": "Cytochrome b-c1 complex subunit Rieske, mitochondrial",
  "gene": "UniProtKB:P47985",
  "gene_symbol": "UQCRFS1",
  "term_id": "GO:0006122",
  "term_label": "mitochondrial electron transport, ubiquinol to cytochrome c"
}